{
  "term_label": "Unknown molecular function",
  "gene_name": "Nuclear pore complex-interacting protein family member B6",
  "gene_symbol": "NPIPB6",
  "term_id": "UNKNOWN:0001",
  "gene": "UniProtKB:E9PJ23"
}